{
  "term_id": "GO:0000724",
  "gene": "UniProtKB:P43351",
  "gene_symbol": "RAD52",
  "gene_name": "DNA repair protein RAD52 homolog",
  "term_label": "double-strand break repair via homologous recombination"
}